{
  "gene_symbol": "TF",
  "term_label": "recycling endosome",
  "gene": "UniProtKB:P02787",
  "term_id": "GO:0055037",
  "gene_name": "Serotransferrin"
}